{
  "gene_name": "HEAT repeat-containing protein 1",
  "term_label": "90S preribosome",
  "gene_symbol": "HEATR1",
  "gene": "UniProtKB:Q9H583",
  "term_id": "GO:0030686"
}